glyoxylate reductase activity [GO:0106345] (molecular function) Relationships: is a type of oxidoreductase activity, acting on the CH-OH group of donors, NAD or NADP as acceptor [GO:0016616] Subtypes: glyoxylate reductase (NADPH) activity [GO:0030267], glyoxylate reductase (NADH) activity [GO:0047964] Definition: Catalysis of the reaction: glycolate + NAD(P)+ = glyoxylate + NAD(P)H. References: PMID:3548703 Sources: GOC:curators